{
  "term_id": "GO:0003723",
  "gene": "UniProtKB:P78346",
  "gene_name": "Ribonuclease P protein subunit p30",
  "term_label": "RNA binding",
  "gene_symbol": "RPP30"
}